{
  "gene_name": "Homeobox protein EMX2",
  "term_id": "GO:0006357",
  "gene_symbol": "EMX2",
  "term_label": "regulation of transcription by RNA polymerase II",
  "gene": "UniProtKB:Q04743"
}